regulation of kainate selective glutamate receptor signaling pathway [GO:0106426] (biological process) References: PMID:12597860 Regulation: negatively regulated by negative regulation of kainate selective glutamate receptor signaling pathway [GO:0106427]; positively regulated by positive regulation of kainate selective glutamate receptor signaling pathway [GO:0106428] Relationships: is a type of regulation of glutamate receptor signaling pathway [GO:1900449]; regulates kainate selective glutamate receptor signaling pathway [GO:0098991] Definition: Any process that modulates the frequency, rate or extent of the kainate selective glutamate receptor signaling pathway. Subtypes: negative regulation of kainate selective glutamate receptor signaling pathway [GO:0106427], positive regulation of kainate selective glutamate receptor signaling pathway [GO:0106428]